{
  "term_id": "UNKNOWN:0003",
  "gene_name": "TM2 domain-containing protein 1",
  "gene": "UniProtKB:Q9BX74",
  "term_label": "Unknown cellular component",
  "gene_symbol": "TM2D1"
}